{
  "term_label": "signal transduction",
  "gene_symbol": "SCUBE3",
  "gene": "UniProtKB:Q8IX30",
  "gene_name": "Signal peptide, CUB and EGF-like domain-containing protein 3",
  "term_id": "GO:0007165"
}